{
  "gene_symbol": "CLUAP1",
  "gene_name": "Clusterin-associated protein 1",
  "gene": "UniProtKB:Q96AJ1",
  "term_id": "GO:0060271",
  "term_label": "cilium assembly"
}